{
  "gene_name": "Collagen alpha-3(IV) chain",
  "term_id": "GO:0005587",
  "gene": "UniProtKB:Q01955",
  "gene_symbol": "COL4A3",
  "term_label": "collagen type IV trimer"
}